peri-centrosomal recycling endosome [GO:0098832] (cellular component) Relationships: is a type of recycling endosome [GO:0055037] References: PMID:19696797, PMID:20820847 Definition: A recycling endosome that is organized around the microtubule organizing center, close to the nucleus. This is the main recycling endosome of most cells. It receives input from the Golgi as well as recycled molecules from early endosomes.